{
  "term_label": "mitochondrion",
  "gene_symbol": "MTCH2",
  "gene": "UniProtKB:Q9Y6C9",
  "gene_name": "Mitochondrial carrier homolog 2",
  "term_id": "GO:0005739"
}